{
  "gene_symbol": "TAF10",
  "term_label": "SAGA complex",
  "term_id": "GO:0000124",
  "gene_name": "Transcription initiation factor TFIID subunit 10",
  "gene": "UniProtKB:Q12962"
}